regulation of acinar cell proliferation [GO:1904697] (biological process) Relationships: is a type of GO:0050678; regulates acinar cell proliferation [GO:1990863] Also known as: regulation of acinic cell proliferation, regulation of acinous cell proliferation References: PMID:9788538 Sources: GOC:TermGenie, GO_REF:0000058 Subtypes: negative regulation of acinar cell proliferation [GO:1904698], positive regulation of acinar cell proliferation [GO:1904699] Definition: Any process that modulates the frequency, rate or extent of acinar cell proliferation.